{
  "term_label": "cellular response to cytokine stimulus",
  "gene_symbol": "IFIT1B",
  "term_id": "GO:0071345",
  "gene": "UniProtKB:Q5T764",
  "gene_name": "Interferon-induced protein with tetratricopeptide repeats 1B"
}